{
  "gene": "UniProtKB:A0A2Z4LIS9",
  "term_label": "response to starvation",
  "gene_name": "Forkhead box protein O3B",
  "term_id": "GO:0042594",
  "gene_symbol": "FOXO3B"
}